{
  "gene_name": "Beta-1,4-galactosyltransferase 5",
  "term_label": "glycoprotein biosynthetic process",
  "term_id": "GO:0009101",
  "gene": "UniProtKB:O43286",
  "gene_symbol": "B4GALT5"
}